{
  "gene": "UniProtKB:P0DPF7",
  "term_id": "GO:0007166",
  "gene_name": "T cell receptor beta variable 6-3",
  "gene_symbol": "TRBV6-3",
  "term_label": "cell surface receptor signaling pathway"
}